organophosphate metabolic process [GO:0019637] (biological process) Relationships: is a type of phosphorus metabolic process [GO:0006793] Also known as: organophosphate metabolism Subtypes: GO:0006002, fructose 2,6-bisphosphate metabolic process [GO:0006003], phosphocreatine metabolic process [GO:0006603], phospholipid metabolic process [GO:0006644], nucleoside phosphate metabolic process [GO:0006753], glucose 1-phosphate metabolic process [GO:0019255], GO:0019283, GO:0019574, GO:0019682, ribose phosphate metabolic process [GO:0019693], GO:0030388, aminophosphonate metabolic process [GO:0033051], thiamine diphosphate metabolic process [GO:0042357], GO:0042822, molybdopterin cofactor metabolic process [GO:0043545], inositol phosphate metabolic process [GO:0043647], organophosphate catabolic process [GO:0046434], glucose 6-phosphate metabolic process [GO:0051156], D-xylulose 5-phosphate metabolic process [GO:0051167], alditol phosphate metabolic process [GO:0052646], chitin catabolic process to fructose 6-phosphate via glucosamine [GO:0052776], GO:0061610, 6-sulfoquinovose(1-) catabolic process to glycerone phosphate and 3-sulfolactaldehyde [GO:0061720], carbamoyl phosphate metabolic process [GO:0070408], organophosphate biosynthetic process [GO:0090407], GO:1900867, GO:2001060, GO:2001289 Sources: ISBN:0198506732 Definition: The chemical reactions and pathways involving organophosphates, any phosphate-containing organic compound.